{
  "term_label": "GTPase activity",
  "term_id": "GO:0003924",
  "gene_symbol": "TSR1",
  "gene": "UniProtKB:Q2NL82",
  "gene_name": "Pre-rRNA-processing protein TSR1 homolog"
}